{
  "gene_name": "Melanoma-associated antigen 2",
  "gene": "UniProtKB:P43356",
  "gene_symbol": "MAGEA2B",
  "term_label": "histone deacetylase binding",
  "term_id": "GO:0042826"
}